{
  "gene_name": "Putative mucosal pentraxin homolog",
  "term_id": "UNKNOWN:0001",
  "term_label": "Unknown molecular function",
  "gene": "UniProtKB:A8MV57",
  "gene_symbol": "MPTX1"
}